{
  "gene": "UniProtKB:Q9UGM1",
  "gene_symbol": "CHRNA9",
  "gene_name": "Neuronal acetylcholine receptor subunit alpha-9",
  "term_label": "chemical synaptic transmission",
  "term_id": "GO:0007268"
}